{
  "gene_symbol": "GNL3L",
  "term_id": "GO:0005730",
  "gene": "UniProtKB:Q9NVN8",
  "gene_name": "Guanine nucleotide-binding protein-like 3-like protein",
  "term_label": "nucleolus"
}